protein deglutathionylation [GO:0080058] (biological process) Definition: The protein modification process in which a glutathione molecule is removed from a protein amino acid by breaking a disulfide linkage. Sources: GOC:tb Also known as: protein amino acid deglutathionylation Relationships: is a type of GO:0036211